{
  "term_id": "GO:0010008",
  "gene_name": "Pleckstrin homology domain-containing family M member 2",
  "gene_symbol": "PLEKHM2",
  "gene": "UniProtKB:Q8IWE5",
  "term_label": "endosome membrane"
}